{
  "term_id": "UNKNOWN:0003",
  "term_label": "Unknown cellular component",
  "gene_symbol": "METTL15P1",
  "gene": "UniProtKB:P0C7V9",
  "gene_name": "Putative methyltransferase-like protein 15P1"
}